{
  "term_id": "GO:0043409",
  "gene_symbol": "DUSP26",
  "term_label": "negative regulation of MAPK cascade",
  "gene_name": "Dual specificity protein phosphatase 26",
  "gene": "UniProtKB:Q9BV47"
}